{
  "term_label": "D-glucose transmembrane transporter activity",
  "gene_symbol": "SLC2A2",
  "term_id": "GO:0055056",
  "gene_name": "Solute carrier family 2, facilitated glucose transporter member 2",
  "gene": "UniProtKB:P11168"
}